{
  "term_id": "GO:0005615",
  "gene": "UniProtKB:P01579",
  "term_label": "extracellular space",
  "gene_symbol": "IFNG",
  "gene_name": "Interferon gamma"
}